{
  "gene_name": "Protein CLN8",
  "gene": "UniProtKB:Q9UBY8",
  "term_label": "phospholipid metabolic process",
  "gene_symbol": "CLN8",
  "term_id": "GO:0006644"
}